{
  "gene_symbol": "CDKL3",
  "term_label": "dendrite extension",
  "term_id": "GO:0097484",
  "gene_name": "Cyclin-dependent kinase-like 3",
  "gene": "UniProtKB:Q8IVW4"
}